{
  "gene_name": "DENN domain-containing protein 3",
  "term_id": "GO:0005085",
  "term_label": "guanyl-nucleotide exchange factor activity",
  "gene": "UniProtKB:A2RUS2",
  "gene_symbol": "DENND3"
}